{
  "term_label": "positive regulation of cell differentiation",
  "gene_symbol": "CCN6",
  "gene": "UniProtKB:O95389",
  "gene_name": "Cellular communication network factor 6",
  "term_id": "GO:0045597"
}